positive regulation of osteoblast proliferation [GO:0033690] (biological process) Definition: Any process that activates or increases the rate or extent of osteoblast proliferation. Sources: GOC:mah Also known as: up regulation of osteoblast proliferation, up-regulation of osteoblast proliferation, upregulation of osteoblast proliferation, activation of osteoblast proliferation, stimulation of osteoblast proliferation Relationships: is a type of positive regulation of cell population proliferation [GO:0008284]; is a type of regulation of osteoblast proliferation [GO:0033688]; RO_0002213 osteoblast proliferation [GO:0033687]